{
  "term_label": "translation reinitiation",
  "gene_symbol": "DENR",
  "term_id": "GO:0002188",
  "gene": "UniProtKB:O43583",
  "gene_name": "Density-regulated protein"
}